{
  "term_label": "Unknown molecular function",
  "term_id": "UNKNOWN:0001",
  "gene": "UniProtKB:Q96DX5",
  "gene_name": "Ankyrin repeat and SOCS box protein 9",
  "gene_symbol": "ASB9"
}